regulation of peroxisome proliferator activated receptor signaling pathway [GO:0035358] (biological process) Sources: GOC:bf Relationships: is a type of regulation of intracellular signal transduction [GO:1902531]; regulates peroxisome proliferator activated receptor signaling pathway [GO:0035357] Subtypes: negative regulation of peroxisome proliferator activated receptor signaling pathway [GO:0035359], positive regulation of peroxisome proliferator activated receptor signaling pathway [GO:0035360] Also known as: regulation of PPAR signaling pathway, regulation of peroxisome proliferator activated receptor signalling pathway, regulation of peroxisome proliferator-activated receptor signaling pathway Definition: Any process that modulates the frequency, rate or extent of the peroxisome proliferator activated receptor signaling pathway.